{
  "gene_symbol": "MYO1H",
  "term_label": "actin filament organization",
  "term_id": "GO:0007015",
  "gene": "UniProtKB:Q8N1T3",
  "gene_name": "Unconventional myosin-Ih"
}